{
  "gene_symbol": "PSEN1",
  "gene": "UniProtKB:P49768",
  "gene_name": "Presenilin-1",
  "term_label": "gamma-secretase complex",
  "term_id": "GO:0070765"
}